{
  "term_label": "long-term synaptic potentiation",
  "gene_name": "Glutamate receptor ionotropic, NMDA 2C",
  "gene_symbol": "GRIN2C",
  "gene": "UniProtKB:Q14957",
  "term_id": "GO:0060291"
}